{
  "gene": "UniProtKB:Q9NRJ7",
  "gene_name": "Protocadherin beta-16",
  "gene_symbol": "PCDHB16",
  "term_id": "GO:0007155",
  "term_label": "cell adhesion"
}